protein aggregate center [GO:0140453] (cellular component) References: PMID:32075773 Also known as: PAC, protein aggregate centre Definition: Reversible aggregate of misfolded proteins and chaperones formed to shield thermosensitive proteins from degradation until conditions allow disaggregation and refolding. Relationships: is a type of intracellular membraneless organelle [GO:0043232]